molybdenum cofactor guanylyltransferase activity [GO:0061603] (molecular function) Definition: Catalysis of the reaction GTP + molybdenum cofactor = diphosphate + guanylyl molybdenum cofactor. Sources: EC:2.7.7.77, GOC:dph Relationships: is a type of guanylyltransferase activity [GO:0070568]